{
  "gene_name": "Small glutamine-rich tetratricopeptide repeat-containing protein beta",
  "term_label": "post-translational protein targeting to endoplasmic reticulum membrane",
  "term_id": "GO:0006620",
  "gene": "UniProtKB:Q96EQ0",
  "gene_symbol": "SGTB"
}